{
  "term_id": "GO:0046512",
  "gene_symbol": "SPTLC2",
  "term_label": "sphingosine biosynthetic process",
  "gene_name": "Serine palmitoyltransferase 2",
  "gene": "UniProtKB:O15270"
}